{
  "term_label": "Unknown cellular component",
  "gene_name": "Eukaryotic translation initiation factor 5A-1",
  "gene": "UniProtKB:P63241",
  "term_id": "UNKNOWN:0003",
  "gene_symbol": "EIF5A"
}